erythrocyte aggregation [GO:0034117] (biological process) Relationships: is a type of homotypic cell-cell adhesion [GO:0034109] Also known as: RBC aggregation, red blood cell aggregation Definition: The adhesion of one erythrocyte to one or more other erythrocytes via adhesion molecules. Regulation: regulated by regulation of erythrocyte aggregation [GO:0034118]; negatively regulated by negative regulation of erythrocyte aggregation [GO:0034119]; positively regulated by positive regulation of erythrocyte aggregation [GO:0034120] References: PMID:14631543 Sources: GOC:add